{
  "gene_name": "Leucine repeat adapter protein 25",
  "term_label": "lamellipodium",
  "gene": "UniProtKB:Q8N5H3",
  "gene_symbol": "FAM89B",
  "term_id": "GO:0030027"
}